epithelial cell proliferation involved in Malpighian tubule morphogenesis [GO:0061331] (BP) Definition: The multiplication or reproduction of epithelial cells, resulting in the expansion of a cell population and contributing to the shaping of a Malpighian tubule. References: PMID:19783135 Sources: GOC:dph, GOC:mtg_kidney_jan10 Relationships: is a type of epithelial cell proliferation involved in renal tubule morphogenesis [GO:2001013]; is part of Malpighian tubule morphogenesis [GO:0007443]